{
  "gene_symbol": "SLC16A6",
  "gene_name": "Monocarboxylate transporter 7",
  "term_id": "GO:0005886",
  "term_label": "plasma membrane",
  "gene": "UniProtKB:O15403"
}